{
  "gene_symbol": "ARMH1",
  "term_id": "UNKNOWN:0003",
  "gene_name": "Armadillo-like helical domain containing protein 1",
  "term_label": "Unknown cellular component",
  "gene": "UniProtKB:Q6PIY5"
}